{
  "gene_name": "Polyadenylate-binding protein 1-like 2",
  "term_label": "cytoplasmic stress granule",
  "gene_symbol": "PABPC1L2A",
  "gene": "UniProtKB:Q5JQF8",
  "term_id": "GO:0010494"
}